5-methyldeoxycytidine-5'-phosphate kinase activity [GO:0047336] (molecular function) Definition: Catalysis of the reaction: 2'-deoxy-5-methyl-5'-cytidylate + ATP = 5-methyldeoxycytidine diphosphate + ADP + H+. Also known as: ATP:5-methyldeoxycytidine-5'-phosphate phosphotransferase activity Relationships: is a type of GO:0016301; is a type of phosphotransferase activity, phosphate group as acceptor [GO:0016776] Sources: EC:2.7.4.19, RHEA:11396